{
  "gene_name": "Vesicular glutamate transporter 2",
  "gene": "UniProtKB:Q9P2U8",
  "gene_symbol": "SLC17A6",
  "term_label": "neurotransmitter transmembrane transporter activity",
  "term_id": "GO:0005326"
}